{
  "term_label": "extracellular space",
  "gene": "UniProtKB:Q9BQB4",
  "term_id": "GO:0005615",
  "gene_symbol": "SOST",
  "gene_name": "Sclerostin"
}